post-anal tail morphogenesis [GO:0036342] (BP) Sources: GOC:bf, GOC:kmv, Wikipedia:Chordate Definition: The process in which a post-anal tail is generated and organized. A post-anal tail is a muscular region of the body that extends posterior to the anus. The post-anal tail may aid locomotion and balance. Relationships: is_a GO:0009653